detection of visible light [GO:0009584] (biological process) Also known as: perception of visible light Subtypes: GO:0007603 Definition: The series of events in which a visible light stimulus is received by a cell and converted into a molecular signal. A visible light stimulus is electromagnetic radiation that can be perceived visually by an organism; for organisms lacking a visual system, this can be defined as light with a wavelength within the range 380 to 780 nm. Relationships: is a type of detection of light stimulus [GO:0009583] Sources: GOC:go_curators, ISBN:0198506732